{
  "gene": "UniProtKB:P16885",
  "term_label": "phosphatidylinositol-4,5-bisphosphate phospholipase C activity",
  "term_id": "GO:0004435",
  "gene_name": "1-phosphatidylinositol 4,5-bisphosphate phosphodiesterase gamma-2",
  "gene_symbol": "PLCG2"
}